{
  "gene": "UniProtKB:Q9BR39",
  "gene_name": "Junctophilin-2",
  "gene_symbol": "JPH2",
  "term_id": "UNKNOWN:0002",
  "term_label": "Unknown biological process"
}